solute:sodium symporter activity [GO:0015370] (molecular function) Also known as: proline/glycine/betaine:hydrogen/sodium symporter activity Definition: Enables the transfer of a solute or solutes from one side of a membrane to the other according to the reaction: solute(out) + Na+(out) = solute(in) + Na+(in). Relationships: is a type of sodium ion transmembrane transporter activity [GO:0015081]; is a type of solute:monoatomic cation symporter activity [GO:0015294] Subtypes: amino acid:sodium symporter activity [GO:0005283], choline:sodium symporter activity [GO:0005307], neurotransmitter:sodium symporter activity [GO:0005328], GO:0005343, myo-inositol:sodium symporter activity [GO:0005367], D-glucose:sodium symporter activity [GO:0005412], nucleoside:sodium symporter activity [GO:0005415], sodium:phosphate symporter activity [GO:0005436], sodium:bicarbonate symporter activity [GO:0008510], GO:0008523, GO:0009674, galactose:sodium symporter activity [GO:0015371], monoatomic anion:sodium symporter activity [GO:0015373], sodium:sulfate symporter activity [GO:0015382], purine-specific nucleoside:sodium symporter activity [GO:0015390], urea:sodium symporter activity [GO:0015401], melibiose:sodium symporter activity [GO:0043887], sodium:galactoside symporter activity [GO:0044669], lysophospholipid:sodium symporter activity [GO:0051978], mannose:sodium symporter activity [GO:0140929], fructose:sodium symporter activity [GO:0140930] Sources: GOC:ai